{
  "gene_symbol": "DUSP1",
  "term_label": "cytoplasm",
  "term_id": "GO:0005737",
  "gene_name": "Dual specificity protein phosphatase 1",
  "gene": "UniProtKB:P28562"
}